deoxycytidine kinase activity [GO:0004137] (molecular function) Also known as: 2'-deoxycytidine kinase activity, Ara-C kinase activity, NTP:deoxycytidine 5'-phosphotransferase activity, arabinofuranosylcytosine kinase activity, deoxycytidine kinase (phosphorylating), deoxycytidine-cytidine kinase activity Sources: EC:2.7.1.74 Relationships: is a type of deoxynucleoside kinase activity [GO:0019136] Definition: Catalysis of the reaction: NTP + deoxycytidine = NDP + CMP.